{
  "gene_name": "Single-stranded DNA-binding protein, mitochondrial",
  "gene": "UniProtKB:Q04837",
  "gene_symbol": "SSBP1",
  "term_id": "GO:0090297",
  "term_label": "positive regulation of mitochondrial DNA replication"
}